{
  "gene": "UniProtKB:Q9HCM3",
  "term_label": "Unknown cellular component",
  "gene_symbol": "KIAA1549",
  "term_id": "UNKNOWN:0003",
  "gene_name": "UPF0606 protein KIAA1549"
}